{
  "term_label": "C-C chemokine receptor activity",
  "term_id": "GO:0016493",
  "gene_symbol": "CXCR4",
  "gene_name": "C-X-C chemokine receptor type 4",
  "gene": "UniProtKB:P61073"
}